{
  "gene": "UniProtKB:Q96F24",
  "gene_name": "Nuclear receptor-binding factor 2",
  "term_label": "autophagy",
  "gene_symbol": "NRBF2",
  "term_id": "GO:0006914"
}